anaerobic cellulose catabolic process [GO:1990488] (biological process) Definition: The chemical reactions and pathways resulting in the breakdown of cellulose, a linear beta1-4 glucan of molecular mass 50-400 kDa with the pyranose units in the -4C1 conformation, in absence of oxygen. References: PMID:8561466 Sources: GOC:mengo_curators Also known as: anaerobic cellulose degradation Relationships: is a type of GO:0030245